{
  "gene_name": "TBC1 domain family member 28",
  "term_id": "UNKNOWN:0002",
  "gene_symbol": "TBC1D28",
  "term_label": "Unknown biological process",
  "gene": "UniProtKB:Q2M2D7"
}